negative regulation of hair follicle placode formation [GO:0061170] (biological process) Definition: Any process that decreases the rate, frequency, or extent of hair follicle placode formation, the developmental process in which a hair placode forms. An hair follicle placode is a thickening of the ectoderm that will give rise to the hair follicle bud. Relationships: is a type of negative regulation of hair follicle development [GO:0051799]; is a type of GO:0061168; negatively regulates hair follicle placode formation [GO:0060789] Sources: GOC:dph